junctional sarcoplasmic reticulum membrane [GO:0014701] (cellular component) Relationships: is a type of sarcoplasmic reticulum membrane [GO:0033017] Sources: GOC:mtg_muscle Definition: The part of the sarcoplasmic reticulum membrane that contains calcium release channels, is devoted to calcium release and is juxtaposed to transverse tubule membrane. The junctional sarcoplasmic reticulum membrane consists of the junctional region of the terminal cisterna membrane.